ethylene receptor histidine kinase activity [GO:0038200] (molecular function) Definition: Combining with ethylene and transmitting the signal within the cell to initiate a change in cell activity by catalysis of the reaction: ATP + a protein-L-histidine = ADP + a protein-L-histidine phosphate. References: PMID:22467798 Sources: GOC:signaling Relationships: is_a GO:0038199; has part protein histidine kinase activity [GO:0004673]